{
  "gene_name": "L-selectin",
  "term_id": "GO:0016339",
  "gene_symbol": "SELL",
  "gene": "UniProtKB:P14151",
  "term_label": "calcium-dependent cell-cell adhesion"
}